{
  "term_label": "cilium assembly",
  "gene_name": "Centrosomal protein of 164 kDa",
  "term_id": "GO:0060271",
  "gene": "UniProtKB:Q9UPV0",
  "gene_symbol": "CEP164"
}